{
  "gene": "UniProtKB:Q00978",
  "term_label": "DNA-binding transcription factor activity, RNA polymerase II-specific",
  "gene_name": "Interferon regulatory factor 9",
  "term_id": "GO:0000981",
  "gene_symbol": "IRF9"
}